{
  "gene": "UniProtKB:Q8NH03",
  "term_id": "GO:0004984",
  "term_label": "olfactory receptor activity",
  "gene_symbol": "OR2T3",
  "gene_name": "Olfactory receptor 2T3"
}